{
  "term_id": "GO:0070506",
  "gene_symbol": "ILDR1",
  "gene": "UniProtKB:Q86SU0",
  "term_label": "high-density lipoprotein particle receptor activity",
  "gene_name": "Immunoglobulin-like domain-containing receptor 1"
}